regulation of skeletal muscle satellite cell proliferation [GO:0014842] (biological process) Definition: Any process that modulates the frequency, rate or extent of skeletal muscle satellite cell proliferation. References: PMID:16607119 Sources: GOC:ef, GOC:mtg_muscle Relationships: is a type of regulation of skeletal muscle cell proliferation [GO:0014857]; regulates skeletal muscle satellite cell proliferation [GO:0014841] Subtypes: growth factor dependent regulation of skeletal muscle satellite cell proliferation [GO:0014843], negative regulation of skeletal muscle satellite cell proliferation [GO:1902723], positive regulation of skeletal muscle satellite cell proliferation [GO:1902724]